{
  "gene_name": "Intestine-specific homeobox",
  "term_label": "neuron development",
  "gene_symbol": "ISX",
  "gene": "UniProtKB:Q2M1V0",
  "term_id": "GO:0048666"
}